cellular response to selenium ion [GO:0071291] (biological process) Definition: Any process that results in a change in state or activity of a cell (in terms of movement, secretion, enzyme production, gene expression, etc.) as a result of a stimulus from selenium ion. Relationships: is a type of response to selenium ion [GO:0010269]; is a type of GO:0071248 Sources: GOC:mah